{
  "gene_name": "Cytochrome P450 2A13",
  "gene": "UniProtKB:Q16696",
  "term_id": "GO:0019373",
  "term_label": "epoxygenase P450 pathway",
  "gene_symbol": "CYP2A13"
}